medial motor column neuron differentiation [GO:0021526] (biological process) Definition: The process in which differentiating motor neurons in the neural tube acquire the specialized structural and/or functional features of medial motor column neurons. Medial motor column neurons are generated at all rostrocaudal levels and send axons to the axial muscles (medial group) and to the body wall muscles (lateral group). Differentiation includes the processes involved in commitment of a cell to a specific fate. References: PMID:11262869 Sources: GOC:cls, GOC:dgh, GOC:dph, GOC:jid, GO_REF:0000021 Relationships: is a type of cell differentiation in spinal cord [GO:0021515]; is a type of neuron differentiation [GO:0030182]; is part of somatic motor neuron differentiation [GO:0021523]